{
  "gene": "UniProtKB:O60242",
  "term_label": "synaptic cleft",
  "gene_symbol": "ADGRB3",
  "gene_name": "Adhesion G protein-coupled receptor B3",
  "term_id": "GO:0043083"
}